{
  "gene_name": "Putative 3-phosphoinositide-dependent protein kinase 2",
  "term_id": "GO:0004674",
  "term_label": "protein serine/threonine kinase activity",
  "gene_symbol": "PDPK2P",
  "gene": "UniProtKB:Q6A1A2"
}